evoked neurotransmitter secretion [GO:0061670] (biological process) Definition: Neurotransmitter secretion that occurs in the presence of the action of a secretagogue or a presynaptic action potential. Relationships: is a type of neurotransmitter secretion [GO:0007269] References: PMID:21334193 Sources: GOC:PARL, GOC:dph, GOC:pad Also known as: stimulus-dependant neurotransmitter secretion